{
  "term_id": "GO:0006355",
  "gene_symbol": "ZNF479",
  "gene": "UniProtKB:Q96JC4",
  "gene_name": "Zinc finger protein 479",
  "term_label": "regulation of DNA-templated transcription"
}